central B cell deletion [GO:0002342] (biological process) Definition: The deletion of B cells by apoptotic process occurring as part of central tolerance induction and B cell selection. Also known as: central B lymphocyte deletion, central B-cell deletion, central B-lymphocyte deletion Sources: GOC:add, GOC:jal, GOC:mtg_apoptosis Regulation: regulated by regulation of central B cell deletion [GO:0002898]; negatively regulated by negative regulation of central B cell deletion [GO:0002899]; positively regulated by positive regulation of central B cell deletion [GO:0002900] Relationships: is a type of B cell deletion [GO:0002516]; is_a programmed cell death involved in cell development [GO:0010623]; is part of central B cell selection [GO:0002340]; BFO_0000050 central B cell tolerance induction [GO:0002510]